{
  "term_id": "GO:0030198",
  "gene": "UniProtKB:Q9Y215",
  "gene_symbol": "COLQ",
  "gene_name": "Acetylcholinesterase collagenic tail peptide",
  "term_label": "extracellular matrix organization"
}